apoptotic process involved in outflow tract morphogenesis [GO:0003275] (biological process) Sources: GOC:mtg_apoptosis, GOC:mtg_heart Also known as: apoptosis involved in outflow tract morphogenesis Relationships: is a type of apoptotic process involved in heart morphogenesis [GO:0003278]; is part of outflow tract morphogenesis [GO:0003151] Regulation: regulated by GO:1902256; negatively regulated by negative regulation of apoptotic process involved in outflow tract morphogenesis [GO:1902257]; positively regulated by positive regulation of apoptotic process involved in outflow tract morphogenesis [GO:1902258] Definition: Any apoptotic process that contributes to the shaping of the outflow tract. The outflow tract is the portion of the heart through which blood flows into the arteries.